{
  "gene_name": "Ras and Rab interactor 3",
  "term_label": "small GTPase binding",
  "gene_symbol": "RIN3",
  "term_id": "GO:0031267",
  "gene": "UniProtKB:Q8TB24"
}